meiotic telomere maintenance via semi-conservative replication [GO:1902989] (biological process) Also known as: telomeric fork progression involved in meiotic cell cycle, telomeric replication fork progression involved in meiotic cell cycle, equal telomere replication involved in meiotic cell cycle Relationships: is a type of telomere maintenance via semi-conservative replication [GO:0032201]; is a type of GO:0070192 Sources: GOC:TermGenie, GO_REF:0000060 Definition: Any telomere maintenance via semi-conservative replication that is involved in meiotic cell cycle.